{
  "gene_symbol": "CYP27C1",
  "term_id": "GO:0061898",
  "term_label": "all-trans retinoic acid 3,4-desaturase activity",
  "gene": "UniProtKB:Q4G0S4",
  "gene_name": "Cytochrome P450 27C1"
}